{
  "gene_name": "AP-2 complex subunit alpha-1",
  "gene_symbol": "AP2A1",
  "gene": "UniProtKB:O95782",
  "term_label": "clathrin-dependent endocytosis",
  "term_id": "GO:0072583"
}